positive regulation of endothelial cell chemotaxis to fibroblast growth factor [GO:2000546] (BP) Relationships: is a type of positive regulation of cell chemotaxis to fibroblast growth factor [GO:1904849]; is a type of regulation of endothelial cell chemotaxis to fibroblast growth factor [GO:2000544]; is a type of positive regulation of endothelial cell chemotaxis [GO:2001028]; positively regulates GO:0035768 Sources: GOC:obol Definition: Any process that activates or increases the frequency, rate or extent of endothelial cell chemotaxis to fibroblast growth factor.